{
  "gene": "UniProtKB:P05112",
  "term_id": "GO:0045893",
  "term_label": "positive regulation of DNA-templated transcription",
  "gene_name": "Interleukin-4",
  "gene_symbol": "IL4"
}